{
  "gene": "UniProtKB:Q8IVQ6",
  "gene_symbol": "ZDHHC21",
  "term_label": "Golgi apparatus",
  "gene_name": "Palmitoyltransferase ZDHHC21",
  "term_id": "GO:0005794"
}